{
  "gene": "UniProtKB:O60313",
  "gene_symbol": "OPA1",
  "term_label": "mitochondrial intermembrane space",
  "term_id": "GO:0005758",
  "gene_name": "Dynamin-like 120 kDa protein, mitochondrial"
}